outer mitochondrial membrane protein complex [GO:0098799] (cellular component) Definition: Any protein complex that is part of the outer mitochondrial membrane. Sources: GOC:dos Subtypes: mitochondrial outer membrane translocase complex [GO:0005742], ERMES complex [GO:0032865], Cdc48p-Npl4p-Vms1p AAA ATPase complex [GO:0036266], MIM complex [GO:0140595] Relationships: is a type of membrane protein complex [GO:0098796]; is a type of mitochondrial protein-containing complex [GO:0098798]; is part of mitochondrial outer membrane [GO:0005741]